{
  "gene_symbol": "GRB10",
  "term_label": "negative regulation of Wnt signaling pathway",
  "gene_name": "Growth factor receptor-bound protein 10",
  "term_id": "GO:0030178",
  "gene": "UniProtKB:Q13322"
}